{
  "term_id": "GO:0005793",
  "gene_name": "Vesicular integral-membrane protein VIP36",
  "term_label": "endoplasmic reticulum-Golgi intermediate compartment",
  "gene_symbol": "LMAN2",
  "gene": "UniProtKB:Q12907"
}